{
  "term_label": "Golgi to secretory granule transport",
  "gene_symbol": "CDR2L",
  "gene": "UniProtKB:Q86X02",
  "gene_name": "Cerebellar degeneration-related protein 2-like",
  "term_id": "GO:0055107"
}